{
  "gene": "UniProtKB:Q9NR09",
  "term_label": "trans-Golgi network",
  "term_id": "GO:0005802",
  "gene_symbol": "BIRC6",
  "gene_name": "Baculoviral IAP repeat-containing protein 6"
}